{
  "gene_name": "Putative protein FAM90A2P",
  "term_id": "UNKNOWN:0003",
  "term_label": "Unknown cellular component",
  "gene": "UniProtKB:Q658T7",
  "gene_symbol": "FAM90A2P"
}